indole catabolic process [GO:0042433] (biological process) Definition: The chemical reactions and pathways resulting in the breakdown of indole (2,3-benzopyrrole), the basis of many biologically active substances (e.g. serotonin, tryptophan). Sources: GOC:jl Relationships: is a type of GO:0042431; is a type of GO:0042436 Also known as: indole breakdown, indole catabolism, indole degradation